{
  "gene": "UniProtKB:Q4KMQ2",
  "term_id": "GO:0005227",
  "term_label": "calcium-activated cation channel activity",
  "gene_symbol": "ANO6",
  "gene_name": "Anoctamin-6"
}